{
  "term_label": "cytoplasm",
  "gene": "UniProtKB:Q96PU5",
  "term_id": "GO:0005737",
  "gene_symbol": "NEDD4L",
  "gene_name": "E3 ubiquitin-protein ligase NEDD4-like"
}